supramolecular polymer [GO:0099081] (cellular component) Relationships: is a type of supramolecular complex [GO:0099080] Definition: A polymeric supramolecular structure. Sources: GOC:dos Subtypes: supramolecular fiber [GO:0099512]